{
  "gene_name": "Olfactory receptor 10H3",
  "term_id": "GO:0005886",
  "gene": "UniProtKB:O60404",
  "gene_symbol": "OR10H3",
  "term_label": "plasma membrane"
}